{
  "term_label": "pore-forming activity",
  "gene_symbol": "DEFA5",
  "gene_name": "Defensin alpha 5",
  "gene": "UniProtKB:Q01523",
  "term_id": "GO:0140911"
}